{
  "gene": "UniProtKB:O95185",
  "term_label": "Unknown cellular component",
  "term_id": "UNKNOWN:0003",
  "gene_name": "Netrin receptor UNC5C",
  "gene_symbol": "UNC5C"
}